alpha5-beta1 integrin-fibronectin-NOV complex [GO:0071117] (cellular component) Relationships: is a type of GO:0098797 References: PMID:12902636 Also known as: ITGA5-ITGB1-FN-1-NOV complex Definition: A protein complex that consists of an alpha5-beta1 integrin complex bound to fibronectin and the extracellular matrix protein NOV.